{
  "gene_name": "BMP and activin membrane-bound inhibitor homolog",
  "term_label": "transforming growth factor beta receptor signaling pathway",
  "gene_symbol": "BAMBI",
  "gene": "UniProtKB:Q13145",
  "term_id": "GO:0007179"
}